euchromatin [GO:0000791] (cellular component) Also known as: transcriptionally active chromatin, nuclear euchromatin Relationships: is a type of chromatin [GO:0000785] Definition: A dispersed and relatively uncompacted form of chromatin that is in a transcription-competent conformation. References: PMID:32017156